propionate metabolic process, methylmalonyl pathway [GO:0019678] (biological process) Also known as: propionate metabolism, methylmalonyl pathway Sources: GOC:go_curators Definition: The chemical reactions and pathways involving propionate that occur in the methylmalonyl pathway. Relationships: is a type of propionate metabolic process [GO:0019541]